bleb [GO:0032059] (cellular component) Definition: A cell extension caused by localized decoupling of the cytoskeleton from the plasma membrane and characterized by rapid formation, rounded shape, and scarcity of organelles within the protrusion. Blebs are formed during apoptosis and other cellular processes, including cell locomotion, cell division, and as a result of physical or chemical stresses. Also known as: plasma membrane bleb References: PMID:12083798, PMID:16624291 Sources: GOC:mtg_apoptosis, Wikipedia:Bleb_(cell_biology) Relationships: is a type of plasma membrane bounded cell projection [GO:0120025]